{
  "gene": "UniProtKB:Q9BU19",
  "term_id": "GO:0000978",
  "gene_name": "Zinc finger protein 692",
  "gene_symbol": "ZNF692",
  "term_label": "RNA polymerase II cis-regulatory region sequence-specific DNA binding"
}